{
  "gene_symbol": "ACKR3",
  "gene": "UniProtKB:P25106",
  "term_label": "cell chemotaxis",
  "gene_name": "Atypical chemokine receptor 3",
  "term_id": "GO:0060326"
}